{
  "gene_name": "Transforming growth factor beta-1-induced transcript 1 protein",
  "term_id": "GO:0034446",
  "term_label": "substrate adhesion-dependent cell spreading",
  "gene": "UniProtKB:O43294",
  "gene_symbol": "TGFB1I1"
}